{
  "gene": "UniProtKB:Q14CX7",
  "gene_symbol": "NAA25",
  "term_id": "GO:0005737",
  "term_label": "cytoplasm",
  "gene_name": "N-alpha-acetyltransferase 25, NatB auxiliary subunit"
}